{
  "term_label": "acrosomal membrane",
  "gene_name": "Izumo sperm-egg fusion protein 1",
  "gene": "UniProtKB:Q8IYV9",
  "gene_symbol": "IZUMO1",
  "term_id": "GO:0002080"
}